{
  "term_label": "Unknown biological process",
  "gene_symbol": "ARHGEF37",
  "term_id": "UNKNOWN:0002",
  "gene": "UniProtKB:A1IGU5",
  "gene_name": "Rho guanine nucleotide exchange factor 37"
}